{
  "term_label": "cell differentiation",
  "term_id": "GO:0030154",
  "gene": "UniProtKB:P08631",
  "gene_symbol": "HCK",
  "gene_name": "Tyrosine-protein kinase HCK"
}